positive regulation of isotype switching to IgE isotypes [GO:0048295] (biological process) Also known as: positive regulation of class switch recombination to IgE isotypes, positive regulation of class switching to IgE isotypes, positive regulation of isotype switch recombination to IgE isotypes, up regulation of isotype switching to IgE isotypes, up-regulation of isotype switching to IgE isotypes, upregulation of isotype switching to IgE isotypes, activation of isotype switching to IgE isotypes, stimulation of isotype switching to IgE isotypes Subtypes: GO:2000572 Sources: GOC:jid Definition: Any process that activates or increases the frequency, rate or extent of isotype switching to IgE isotypes. Relationships: is a type of positive regulation of isotype switching [GO:0045830]; is a type of regulation of isotype switching to IgE isotypes [GO:0048293]; positively regulates isotype switching to IgE isotypes [GO:0048289]